{
  "gene_name": "Ras association domain-containing protein 1",
  "term_label": "nucleus",
  "gene": "UniProtKB:Q9NS23",
  "gene_symbol": "RASSF1",
  "term_id": "GO:0005634"
}